positive regulation of peptidyl-cysteine S-nitrosylation [GO:2000170] (biological process) Sources: GOC:obol Definition: Any process that activates or increases the frequency, rate or extent of peptidyl-cysteine S-nitrosylation. Relationships: is a type of positive regulation of protein modification process [GO:0031401]; is a type of regulation of peptidyl-cysteine S-nitrosylation [GO:2000169]; positively regulates GO:0018119